{
  "term_id": "UNKNOWN:0001",
  "gene_symbol": "GINS2",
  "term_label": "Unknown molecular function",
  "gene_name": "DNA replication complex GINS protein PSF2",
  "gene": "UniProtKB:Q9Y248"
}